{
  "gene_name": "Uncharacterized protein",
  "gene": "UniProtKB:A0A140TA64",
  "term_id": "UNKNOWN:0003",
  "gene_symbol": "LOC100996750",
  "term_label": "Unknown cellular component"
}